{
  "term_id": "UNKNOWN:0002",
  "gene_symbol": "RPAP3",
  "gene": "UniProtKB:Q9H6T3",
  "gene_name": "RNA polymerase II-associated protein 3",
  "term_label": "Unknown biological process"
}